myeloid dendritic cell differentiation involved in immune response [GO:0002284] (biological process) Relationships: is a type of myeloid dendritic cell activation involved in immune response [GO:0002277]; is a type of GO:0043011 Sources: GOC:add, ISBN:0781735149 Definition: The process in which an immature myeloid dendritic cell acquires the specialized features of a mature myeloid dendritic cell as part of an immune response. Also known as: myeloid dendritic cell differentiation during immune response